mitochondrial RNA catabolic process [GO:0000957] (biological process) Definition: The chemical reactions and pathways resulting in the breakdown of RNA transcribed from the mitochondrial genome and occurring in the mitochondrion. Regulation: regulated by GO:0000960; negatively regulated by GO:0000961; RO_0002213 by positive regulation of mitochondrial RNA catabolic process [GO:0000962] Sources: GOC:krc, GOC:mah Subtypes: mitochondrial mRNA catabolic process [GO:0000958], GO:2000827 Relationships: is a type of mitochondrial RNA metabolic process [GO:0000959]; is a type of RNA catabolic process [GO:0006401]